regulation of telomere capping [GO:1904353] (biological process) Subtypes: negative regulation of telomere capping [GO:1904354], positive regulation of telomere capping [GO:1904355], regulation of protection from non-homologous end joining at telomere [GO:1905764] Also known as: regulation of telomere end protection Relationships: is a type of regulation of telomere maintenance [GO:0032204]; regulates telomere capping [GO:0016233] References: PMID:23959892 Sources: GOC:BHF, GOC:BHF_telomere, GOC:TermGenie, GOC:nc, GO_REF:0000058 Definition: Any process that modulates the frequency, rate or extent of telomere capping.